{
  "gene": "UniProtKB:P59044",
  "gene_name": "NACHT, LRR and PYD domains-containing protein 6",
  "term_label": "canonical inflammasome complex",
  "gene_symbol": "NLRP6",
  "term_id": "GO:0061702"
}